{
  "gene_symbol": "ZBTB2",
  "gene": "UniProtKB:Q8N680",
  "term_id": "GO:0001817",
  "term_label": "regulation of cytokine production",
  "gene_name": "Zinc finger and BTB domain-containing protein 2"
}